{
  "gene": "UniProtKB:Q8IXZ3",
  "term_label": "regulation of transcription by RNA polymerase II",
  "term_id": "GO:0006357",
  "gene_symbol": "SP8",
  "gene_name": "Transcription factor Sp8"
}